actomyosin contractile ring actin filament bundle assembly [GO:0071519] (biological process) Relationships: is_a actin filament bundle assembly [GO:0051017]; is a type of actomyosin contractile ring assembly actin filament organization [GO:2000689] Definition: A process of actin filament bundle formation that occurs in the context of assembling an actomyosin contractile ring during cytokinesis. References: PMID:19713940 Sources: GOC:mah Subtypes: mitotic contractile ring actin filament bundle assembly [GO:1903477] Also known as: actin filament bundle assembly involved in cytokinetic actomyosin contractile ring assembly, actin filament bundle assembly involved in actomyosin contractile ring formation